{
  "term_label": "Unknown biological process",
  "term_id": "UNKNOWN:0002",
  "gene_symbol": "FAM27E3",
  "gene": "UniProtKB:Q08E93",
  "gene_name": "Protein FAM27E3"
}